{
  "gene_symbol": "ZC3H12C",
  "gene": "UniProtKB:Q9C0D7",
  "gene_name": "Probable ribonuclease ZC3H12C",
  "term_label": "RNA endonuclease activity",
  "term_id": "GO:0004521"
}